somatic sex determination [GO:0018993] (biological process) Sources: GOC:ems Definition: The determination of sex and sexual phenotypes in an organism's soma. Relationships: is a type of sex determination [GO:0007530]; is part of GO:0007275 Subtypes: female somatic sex determination [GO:0019101], male somatic sex determination [GO:0019102], GO:0042001